{
  "term_label": "kinesin complex",
  "gene": "UniProtKB:Q9Y496",
  "gene_symbol": "KIF3A",
  "gene_name": "Kinesin-like protein KIF3A",
  "term_id": "GO:0005871"
}